negative regulation of tumor necrosis factor superfamily cytokine production [GO:1903556] (biological process) Definition: Any process that stops, prevents or reduces the frequency, rate or extent of tumor necrosis factor superfamily cytokine production. Subtypes: GO:0032719, negative regulation of tumor necrosis factor production [GO:0032720], negative regulation of lymphotoxin A production [GO:0032721], GO:2000308 References: PMID:24187568 Sources: GOC:TermGenie, GO_REF:0000058 Relationships: is a type of GO:0001818; is a type of regulation of tumor necrosis factor superfamily cytokine production [GO:1903555]; negatively regulates tumor necrosis factor superfamily cytokine production [GO:0071706] Also known as: down regulation of TNFSF cytokine production, down regulation of tumor necrosis factor superfamily cytokine production, down-regulation of TNFSF cytokine production, down-regulation of tumor necrosis factor superfamily cytokine production, downregulation of TNFSF cytokine production, downregulation of tumor necrosis factor superfamily cytokine production, negative regulation of TNFSF cytokine production, inhibition of TNFSF cytokine production, inhibition of tumor necrosis factor superfamily cytokine production, down regulation of TNF superfamily production, down-regulation of TNF superfamily production, downregulation of TNF superfamily production, inhibition of TNF superfamily production, negative regulation of TNF superfamily production